coenzyme M biosynthetic process [GO:0019295] (biological process) Also known as: coenzyme M anabolism, coenzyme M biosynthesis, coenzyme M formation, coenzyme M synthesis Definition: The chemical reactions and pathways resulting in the formation of coenzyme M (2-thioethansulfonate), a coenzyme involved in the utilization of methane by methanogenic prokaryotes. Sources: ISBN:0198547684 Relationships: is a type of organic acid biosynthetic process [GO:0016053]; is a type of GO:0044272